backward locomotion [GO:0043057] (biological process) Definition: Posterior movement of an organism, e.g. following the direction of the tail of an animal. Regulation: regulated by GO:0043058; RO_0002212 by negative regulation of backward locomotion [GO:1905851]; positively regulated by positive regulation of backward locomotion [GO:1905852] Relationships: is a type of directional locomotion [GO:0033058] Sources: GOC:go_curators